{
  "term_label": "Unknown biological process",
  "term_id": "UNKNOWN:0002",
  "gene_name": "Formin-binding protein 1",
  "gene_symbol": "FNBP1",
  "gene": "UniProtKB:Q96RU3"
}